virus receptor activity [GO:0001618] (molecular function) References: PMID:7621403 Sources: GOC:bf, GOC:dph, UniProtKB-KW:KW-1183 Relationships: is_a exogenous protein binding [GO:0140272]; BFO_0000050 symbiont entry into host cell [GO:0046718] Also known as: viral receptor activity Definition: Combining with a virus component and mediating entry of the virus into the cell.